long-chain fatty acyl-CoA binding [GO:0036042] (molecular function) Definition: Binding to a long-chain fatty acyl-CoA, any derivative of coenzyme A in which the sulfhydryl group is in a thioester linkage with a long-chain fatty-acyl group. A long-chain fatty acid has an aliphatic tail containing 13 to 22 carbons. Also known as: long-chain fatty acyl-coenyme A binding Note: While there is not universal consensus on the lengths of short-, medium-, long- and very-long-chain fatty acids, the GO uses the definitions in ChEBI (see CHEBI:26666, CHEBI:59554, CHEBI:15904 and CHEBI:27283). Sources: GOC:krc, GOC:pm Relationships: is a type of fatty-acyl-CoA binding [GO:0000062]